carotene metabolic process [GO:0016119] (BP) Definition: The chemical reactions and pathways involving carotenes, hydrocarbon carotenoids. Sources: ISBN:0198547684 Relationships: is a type of GO:0042214 Also known as: carotene metabolism Subtypes: carotene biosynthetic process [GO:0016120], GO:0016121, 9,9'-di-cis-zeta-carotene desaturation to 7,9,7',9'-tetra-cis-lycopene [GO:0052889], GO:1901810